{
  "gene_name": "Beta-ureidopropionase",
  "term_label": "beta-ureidopropionase activity",
  "gene": "UniProtKB:Q9UBR1",
  "gene_symbol": "UPB1",
  "term_id": "GO:0003837"
}